{
  "gene_name": "FYVE, RhoGEF and PH domain-containing protein 1",
  "gene": "UniProtKB:P98174",
  "term_label": "cytoskeleton organization",
  "gene_symbol": "FGD1",
  "term_id": "GO:0007010"
}